{
  "term_id": "GO:0005737",
  "gene": "UniProtKB:P80511",
  "gene_symbol": "S100A12",
  "gene_name": "Protein S100-A12",
  "term_label": "cytoplasm"
}